regulation of siRNA-independent facultative heterochromatin formation [GO:1902801] (biological process) References: PMID:24210919 Sources: GOC:TermGenie, GO_REF:0000058 Also known as: regulation of heterochromatin island assembly, regulation of heterochromatin island formation, regulation of siRNA-independent facultative heterochromatin assembly Definition: Any process that modulates the frequency, rate or extent of siRNA-independent facultative heterochromatin assembly. Relationships: is a type of regulation of heterochromatin formation [GO:0031445]; regulates siRNA-independent facultative heterochromatin formation [GO:1902794]